pyruvate secondary active transmembrane transporter activity [GO:0005477] (molecular function) Sources: GOC:mtg_transport Definition: Enables the transfer of pyruvate from one side of a membrane to the other, up its concentration gradient. The transporter binds the solute and undergoes a series of conformational changes. Transport works equally well in either direction and is driven by a chemiosmotic source of energy. Secondary active transporters include symporters and antiporters. Also known as: pyruvate carrier activity Relationships: is a type of secondary active monocarboxylate transmembrane transporter activity [GO:0015355]; is a type of GO:0050833